{
  "gene": "UniProtKB:Q6JBY9",
  "gene_name": "CapZ-interacting protein",
  "gene_symbol": "RCSD1",
  "term_label": "protein localization to endosome",
  "term_id": "GO:0036010"
}